{
  "term_label": "Unknown biological process",
  "gene_name": "Thioredoxin",
  "term_id": "UNKNOWN:0002",
  "gene_symbol": "TXN",
  "gene": "UniProtKB:P10599"
}